chlorogenate hydrolase activity [GO:0047745] (molecular function) Sources: EC:3.1.1.42, RHEA:20689 Relationships: is a type of GO:0052689 Definition: Catalysis of the reaction: chlorogenate + H2O = (-)-quinate + cis-caffeate + H+. Also known as: chlorogenase activity, chlorogenic acid esterase activity